{
  "gene_symbol": "PRSS47P",
  "gene": "UniProtKB:A8MTI9",
  "gene_name": "Putative serine protease 47",
  "term_label": "serine-type endopeptidase activity",
  "term_id": "GO:0004252"
}